cysteine synthase activity [GO:0004124] (molecular function) Also known as: cysteine synthase activity, acting on O-acetyl-L-serine, O-acetylserine (thiol)-lyase A activity, 3-O-acetyl-L-serine:hydrogen-sulfide 2-amino-2-carboxyethyltransferase activity, O(3)-acetyl-L-serine acetate-lyase (adding hydrogen-sulfide) activity, O-acetyl-L-serine sulfhydrylase activity, O-acetyl-L-serine sulfohydrolase activity, O-acetylserine (thiol)-lyase activity, O-acetylserine sulfhydrylase activity, O3-acetyl-L-serine acetate-lyase (adding hydrogen-sulfide), O3-acetyl-L-serine:hydrogen-sulfide 2-amino-2-carboxyethyltransferase activity, OAS sulfhydrylase activity, acetylserine sulfhydrylase activity, cysteine synthetase activity Relationships: is a type of transferase activity, transferring alkyl or aryl (other than methyl) groups [GO:0016765]; is part of cysteine biosynthetic process [GO:0019344] Sources: EC:2.5.1.47 Definition: Catalysis of the reaction: O3-acetyl-L-serine + hydrogen sulfide = L-cysteine + acetate.